{
  "term_label": "catenin complex",
  "gene": "UniProtKB:P55287",
  "term_id": "GO:0016342",
  "gene_name": "Cadherin-11",
  "gene_symbol": "CDH11"
}